histone H2A reader activity [GO:0140054] (molecular function) References: PMID:11498575, PMID:25688442, PMID:31082667, PMID:34726351 Also known as: histone H2A reader Definition: A histone reader that specifically binds either to an unmodified histone H2A or a form modified by a post-translational modification on a specific residue. The most common PTMs on histones are methylation, acetylation and phosphorylation. Subtypes: GO:0140120, histone H2AK15ac reader activity [GO:0140126], GO:0140130, histone H2AT120pho reader activity [GO:0140172], histone H2AS139pho reader activity [GO:0140173] Relationships: is a type of histone reader activity [GO:0140566]